{
  "term_label": "thyroxine 5'-deiodinase activity",
  "term_id": "GO:0004800",
  "gene_symbol": "DIO2",
  "gene": "UniProtKB:Q92813",
  "gene_name": "Type II iodothyronine deiodinase"
}